{
  "term_label": "Unknown biological process",
  "term_id": "UNKNOWN:0002",
  "gene_symbol": "MPHOSPH9",
  "gene_name": "M-phase phosphoprotein 9",
  "gene": "UniProtKB:Q99550"
}